sexine [GO:0043673] (cellular component) Relationships: is_a cellular anatomical structure [GO:0110165]; is part of exine [GO:0043668] Definition: The outer, sculptured layer of the exine, which lies above the nexine. References: PMID:5722147 Note: Note that the sexine sometimes consists of 5 layers, but of those, 3 layers are the most common (sexine 1 = columellae; sexine 2 = tectum; sexine 3 = sculpture elements). Sexine is distinguished on purely morphological criteria; compare with 'ectexine ; GO:0043669'. See also 'nexine ; GO:0043672'.